{
  "term_id": "GO:0071363",
  "gene_name": "Serine_threonine-protein kinase receptor R3",
  "term_label": "cellular response to growth factor stimulus",
  "gene_symbol": "ACVRL1",
  "gene": "UniProtKB:P37023"
}